{
  "gene_symbol": "ARL13B",
  "gene": "UniProtKB:Q3SXY8",
  "term_id": "UNKNOWN:0001",
  "gene_name": "ADP-ribosylation factor-like protein 13B",
  "term_label": "Unknown molecular function"
}